{
  "gene_symbol": "NME2",
  "term_id": "UNKNOWN:0003",
  "gene_name": "Nucleoside diphosphate kinase B",
  "term_label": "Unknown cellular component",
  "gene": "UniProtKB:P22392"
}